klinokinesis [GO:0042468] (biological process) Relationships: is a type of GO:0042465 Definition: The movement of a cell or organism in response to a stimulus in which the frequency or magnitude of turning behavior is altered. References: PMID:2790068 Sources: GOC:jl